positive regulation of cholesterol import [GO:1904109] (biological process) References: PMID:16772292 Sources: GOC:TermGenie, GO_REF:0000058 Definition: Any process that activates or increases the frequency, rate or extent of cholesterol import. Also known as: positive regulation of cholesterol uptake, up regulation of cholesterol import, up regulation of cholesterol uptake, up-regulation of cholesterol import, up-regulation of cholesterol uptake, upregulation of cholesterol import, upregulation of cholesterol uptake, activation of cholesterol import, activation of cholesterol uptake Relationships: is a type of positive regulation of cholesterol transport [GO:0032376]; is a type of GO:0060620; positively regulates GO:0070508